{
  "gene_name": "EMILIN-3",
  "gene": "UniProtKB:Q9NT22",
  "term_label": "Unknown biological process",
  "term_id": "UNKNOWN:0002",
  "gene_symbol": "EMILIN3"
}